endo-beta-bergamotene synthase activity [GO:0102061] (MF) Sources: GOC:pz, RHEA:30467 Definition: Catalysis of the reaction: 2-cis,6-cis-farnesyl diphosphate = (+)-endo-beta-bergamotene + diphosphoric acid. Relationships: is a type of carbon-oxygen lyase activity, acting on phosphates [GO:0016838] Also known as: (+)-endo-beta-bergamotene synthase ((2Z,6Z)-farnesyl diphosphate cyclizing), (2Z,6Z)-farnesyl diphosphate = (+)-endo-beta-bergamotene, endo-beta-bergamontene synthase activity